{
  "term_label": "Unknown cellular component",
  "gene": "UniProtKB:O75746",
  "gene_symbol": "SLC25A12",
  "gene_name": "Electrogenic aspartate_glutamate antiporter SLC25A12, mitochondrial",
  "term_id": "UNKNOWN:0003"
}